{
  "gene": "UniProtKB:P21579",
  "term_id": "GO:0005886",
  "gene_symbol": "SYT1",
  "gene_name": "Synaptotagmin-1",
  "term_label": "plasma membrane"
}